{
  "gene": "UniProtKB:Q6NXT6",
  "gene_symbol": "TAPT1",
  "gene_name": "Transmembrane anterior posterior transformation protein 1 homolog",
  "term_label": "Unknown molecular function",
  "term_id": "UNKNOWN:0001"
}